regulation of collateral sprouting in absence of injury [GO:0048696] (biological process) Sources: GOC:dgh, GOC:dph, GOC:jid, GOC:lm Definition: Any process that modulates the frequency, rate or extent of collateral sprouting in the absence of injury. Relationships: is a type of regulation of collateral sprouting [GO:0048670]; regulates collateral sprouting in absence of injury [GO:0048669] Subtypes: positive regulation of collateral sprouting in absence of injury [GO:0048697], negative regulation of collateral sprouting in absence of injury [GO:0048698]